{
  "gene": "UniProtKB:Q7Z4V5",
  "term_id": "GO:0061628",
  "gene_name": "Hepatoma-derived growth factor-related protein 2",
  "gene_symbol": "HDGFL2",
  "term_label": "histone H3K27me3 reader activity"
}